{
  "gene": "UniProtKB:Q8NAJ2",
  "gene_name": "Putative uncharacterized protein encoded by LINC02913",
  "term_label": "Unknown molecular function",
  "gene_symbol": "LINC02913",
  "term_id": "UNKNOWN:0001"
}